cellular response to follicle-stimulating hormone stimulus [GO:0071372] (biological process) Sources: GOC:mah Also known as: cellular response to FSH stimulus, cellular response to follicle stimulating hormone stimulus Definition: Any process that results in a change in state or activity of a cell (in terms of movement, secretion, enzyme production, gene expression, etc.) as a result of a follicle-stimulating hormone stimulus. Relationships: is a type of GO:0032354; is a type of cellular response to gonadotropin stimulus [GO:0071371]